{
  "gene": "UniProtKB:Q9H6X4",
  "gene_symbol": "TMEM134",
  "term_id": "UNKNOWN:0001",
  "term_label": "Unknown molecular function",
  "gene_name": "Transmembrane protein 134"
}